transposable element silencing by piRNA-mediated mRNA destabilization [GO:0141009] (BP) Also known as: piRNA-mediated post-transcriptional retrotransposon silencing, piRNA-mediated retrotransposon silencing by mRNA destabilization References: PMID:22121019 Relationships: is a type of piRNA-mediated gene silencing by mRNA destabilization [GO:0140991]; is a type of transposable element silencing by mRNA destabilization [GO:0141008] Definition: A transposable element silencing mechanism in which mRNAs transcribed from transposons are targeted for degradation by a Piwi-associated RNA (piRNA).